cotyledon vascular tissue pattern formation [GO:0010588] (BP) Relationships: is_a xylem and phloem pattern formation [GO:0010051]; is part of cotyledon morphogenesis [GO:0048826] References: PMID:10559439 Definition: Vascular tissue pattern formation as it occurs in the cotyledon of vascular plants.